{
  "term_label": "Unknown cellular component",
  "term_id": "UNKNOWN:0003",
  "gene_symbol": "EFCAB12",
  "gene": "UniProtKB:Q6NXP0",
  "gene_name": "EF-hand calcium-binding domain-containing protein 12"
}